inner acrosomal membrane [GO:0002079] (cellular component) Definition: The acrosomal membrane region that underlies the acrosomal vesicle and is located toward the sperm nucleus. This region is responsible for molecular interactions allowing the sperm to penetrate the zona pellucida and fuses with the egg plasma membrane. Note: Note that this term is not a descendant of 'organelle inner membrane ; GO:0019866' because the outer acrosomal membrane is a portion of the acrosomal membrane; the latter is a single lipid bilayer. References: PMID:3899643, PMID:8936405 Sources: GOC:dph Relationships: is a type of cytoplasmic vesicle membrane [GO:0030659]; is part of acrosomal membrane [GO:0002080]